host cell smooth endoplasmic reticulum [GO:0044170] (cellular component) Sources: GOC:jl Definition: The irregular network of unit membranes, visible only by electron microscopy, that occurs in the host cell cytoplasm of many eukaryotic cells. The membranes form a complex meshwork of tubular channels, which are often expanded into slitlike cavities called cisternae. The host smooth ER has no ribosomes adhering to the outer surface. Relationships: is a type of host cell endoplasmic reticulum [GO:0044165] Also known as: host smooth endoplasmic reticulum